cytokinin biosynthetic process [GO:0009691] (biological process) Definition: The chemical reactions and pathways resulting in the formation of cytokinins, a class of adenine-derived compounds that can function in plants as growth regulators. Sources: ISBN:0387969845 Also known as: cytokinin anabolism, cytokinin biosynthesis, cytokinin formation, cytokinin synthesis Relationships: is a type of cytokinin metabolic process [GO:0009690]; is a type of hormone biosynthetic process [GO:0042446] Subtypes: zeatin biosynthetic process [GO:0033398], isopentenyl adenine biosynthetic process [GO:0034265], discadenine biosynthetic process [GO:0034268]